{
  "term_id": "GO:0046703",
  "gene_symbol": "RAET1E",
  "term_label": "natural killer cell lectin-like receptor binding",
  "gene_name": "Retinoic acid early transcript 1E",
  "gene": "UniProtKB:Q8TD07"
}